{
  "term_label": "norepinephrine biosynthetic process",
  "gene_symbol": "MOXD1",
  "gene": "UniProtKB:Q6UVY6",
  "term_id": "GO:0042421",
  "gene_name": "DBH-like monooxygenase protein 1"
}